{
  "term_id": "UNKNOWN:0001",
  "gene_symbol": "TSPAN33",
  "gene": "UniProtKB:Q86UF1",
  "term_label": "Unknown molecular function",
  "gene_name": "Tetraspanin-33"
}